aryl-alcohol oxidase activity [GO:0047682] (molecular function) Definition: Catalysis of the reaction: an aromatic primary alcohol + O2 = an aromatic aldehyde + H2O2. Also known as: veratryl alcohol oxidase activity, arom. alcohol oxidase activity, aryl alcohol oxidase activity, aryl-alcohol:oxygen oxidoreductase activity Sources: EC:1.1.3.7, MetaCyc:ARYL-ALCOHOL-OXIDASE-RXN Relationships: is a type of oxidoreductase activity, acting on the CH-OH group of donors, oxygen as acceptor [GO:0016899]